{
  "gene": "UniProtKB:Q6ZST4",
  "gene_name": "Lipocalin-like 1 protein",
  "term_id": "UNKNOWN:0001",
  "term_label": "Unknown molecular function",
  "gene_symbol": "LCNL1"
}